{
  "gene_name": "SLAIN motif-containing protein 1",
  "gene": "UniProtKB:Q8ND83",
  "term_id": "UNKNOWN:0001",
  "term_label": "Unknown molecular function",
  "gene_symbol": "SLAIN1"
}